{
  "gene_symbol": "MESP2",
  "term_label": "somite rostral/caudal axis specification",
  "term_id": "GO:0032525",
  "gene_name": "Mesoderm posterior protein 2",
  "gene": "UniProtKB:Q0VG99"
}